{
  "gene_name": "Cyclin-dependent kinase 4 inhibitor C",
  "gene_symbol": "CDKN2C",
  "term_id": "GO:0005737",
  "gene": "UniProtKB:P42773",
  "term_label": "cytoplasm"
}